{
  "term_id": "GO:0007030",
  "gene": "UniProtKB:Q92538",
  "term_label": "Golgi organization",
  "gene_name": "Golgi-specific brefeldin A-resistance guanine nucleotide exchange factor 1",
  "gene_symbol": "GBF1"
}